{
  "term_id": "GO:1901907",
  "gene_name": "Diphosphoinositol polyphosphate phosphohydrolase 2",
  "gene": "UniProtKB:Q9NZJ9",
  "term_label": "diadenosine pentaphosphate catabolic process",
  "gene_symbol": "NUDT4"
}